{
  "gene": "UniProtKB:Q9H3N8",
  "term_label": "plasma membrane",
  "gene_symbol": "HRH4",
  "gene_name": "Histamine H4 receptor",
  "term_id": "GO:0005886"
}